{
  "gene_symbol": "TTC7A",
  "gene": "UniProtKB:Q9ULT0",
  "gene_name": "Tetratricopeptide repeat protein 7A",
  "term_id": "UNKNOWN:0001",
  "term_label": "Unknown molecular function"
}